single-species biofilm formation on inanimate substrate [GO:0044011] (biological process) Sources: GOC:cc Relationships: is a type of single-species submerged biofilm formation [GO:0090609] Regulation: RO_0002211 by regulation of single-species biofilm formation on inanimate substrate [GO:1900231]; negatively regulated by negative regulation of single-species biofilm formation on inanimate substrate [GO:1900232]; positively regulated by GO:1900233 Definition: A process in which microorganisms of the same species attach to and grow on an inanimate surface such as a rock or pipe, and produce extracellular polymers that facilitate attachment and matrix formation, resulting in an alteration in the phenotype of the organisms with respect to growth rate and gene transcription.